ventral trunk neural crest cell migration [GO:0036486] (biological process) Also known as: trunk NCC migration through anterior sclerotome, trunk NCC migration within somite, ventral trunk NCC migration References: PMID:16319111, PMID:19386662 Sources: GOC:PARL, GOC:bf, GOC:mat Relationships: is a type of trunk neural crest cell migration [GO:0036484] Definition: The movement of trunk neural crest cells from the neural tube, travelling ventrally through the anterior half of each sclerotome. Trunk neural crest cells that remain in the sclerotome form the dorsal root ganglia containing the sensory neurons. Trunk neural crest cells that continue more ventrally form the sympathetic ganglia, the adrenal medulla, and the nerve clusters surrounding the aorta.